synaptic membrane [GO:0097060] (cellular component) Definition: A specialized area of membrane on either the presynaptic or the postsynaptic side of a synapse, the junction between a nerve fiber of one neuron and another neuron or muscle fiber or glial cell. Subtypes: dendritic spine membrane [GO:0032591], presynaptic periactive zone [GO:0036062], presynaptic membrane [GO:0042734], postsynaptic membrane [GO:0045211], presynaptic active zone membrane [GO:0048787], presynaptic endocytic zone membrane [GO:0098835], postsynaptic endocytic zone membrane [GO:0098844], postsynaptic specialization membrane [GO:0099634] Relationships: is a type of plasma membrane region [GO:0098590]; is part of synapse [GO:0045202] References: PMID:20410104 Sources: GOC:BHF